{
  "term_id": "GO:0005634",
  "gene": "UniProtKB:P51532",
  "gene_name": "Transcription activator BRG1",
  "term_label": "nucleus",
  "gene_symbol": "SMARCA4"
}